cochlear outer hair cell electromotile response [GO:0099129] (BP) Definition: A rapid, force generating length change of an outer hair cell in response to electrical stimulation. This occurs naturally as during hearing where it serves a source of mechanical amplification. References: PMID:12239568, PMID:16887876, PMID:2187727 Relationships: is a type of GO:0070252